regulation of ribosomal subunit export from nucleus [GO:2000200] (biological process) Definition: Any process that modulates the frequency, rate or extent of ribosomal subunit export from nucleus. Relationships: is a type of GO:0046822; is a type of regulation of ribonucleoprotein complex localization [GO:2000197]; regulates GO:0000054 Subtypes: GO:2000201, positive regulation of ribosomal subunit export from nucleus [GO:2000202], regulation of ribosomal large subunit export from nucleus [GO:2000203], regulation of ribosomal small subunit export from nucleus [GO:2000206] Also known as: regulation of ribosomal subunit export from cell nucleus, regulation of ribosomal subunit export out of nucleus, regulation of ribosomal subunit transport from nucleus to cytoplasm, regulation of ribosomal subunit-nucleus export, regulation of ribosome export from nucleus Sources: GOC:mah